{
  "gene_name": "Probable ubiquitin carboxyl-terminal hydrolase FAF-Y",
  "gene": "UniProtKB:O00507",
  "term_id": "GO:0005634",
  "term_label": "nucleus",
  "gene_symbol": "USP9Y"
}